{
  "gene_symbol": "CLEC2A",
  "term_id": "GO:0009897",
  "gene": "UniProtKB:Q6UVW9",
  "gene_name": "C-type lectin domain family 2 member A",
  "term_label": "external side of plasma membrane"
}